mesenchymal cell proliferation involved in lung development [GO:0060916] (biological process) Relationships: is a type of mesenchymal cell proliferation [GO:0010463]; is part of lung development [GO:0030324] Definition: The multiplication or reproduction of cells, resulting in the expansion of a mesenchymal cell population that contributes to the progression of the lung over time. A mesenchymal cell is a cell that normally gives rise to other cells that are organized as three-dimensional masses, rather than sheets. Sources: GOC:dph Regulation: regulated by regulation of mesenchymal cell proliferation involved in lung development [GO:2000790]; negatively regulated by negative regulation of mesenchymal cell proliferation involved in lung development [GO:2000791]; positively regulated by GO:2000792